asymmetric cell division [GO:0008356] (biological process) Definition: The asymmetric division of cells to produce two daughter cells with different developmental potentials. It is of fundamental significance for the generation of cell diversity. References: PMID:11672519 Subtypes: cystoblast division [GO:0007282], zygote asymmetric cell division [GO:0010070], sensory organ precursor cell division [GO:0045035], GO:0055059, asymmetric stem cell division [GO:0098722] Regulation: regulated by regulation of asymmetric cell division [GO:0009786]; negatively regulated by negative regulation of asymmetric cell division [GO:0045769]; positively regulated by positive regulation of asymmetric cell division [GO:0045770] Also known as: asymmetrical cell division, asymmetric cytokinesis, asymmetrical cytokinesis Relationships: is a type of cell division [GO:0051301]